{
  "gene_name": "Transmembrane protein 222",
  "gene": "UniProtKB:Q9H0R3",
  "term_id": "UNKNOWN:0003",
  "term_label": "Unknown cellular component",
  "gene_symbol": "TMEM222"
}